{
  "term_label": "protein-containing complex",
  "gene_name": "Organic solute transporter subunit beta",
  "gene": "UniProtKB:Q86UW2",
  "term_id": "GO:0032991",
  "gene_symbol": "SLC51B"
}